{
  "gene_name": "Dynein regulatory complex subunit 2",
  "term_id": "GO:0005930",
  "gene": "UniProtKB:Q8IXS2",
  "gene_symbol": "CCDC65",
  "term_label": "axoneme"
}